{
  "gene": "UniProtKB:Q5T036",
  "term_label": "Unknown biological process",
  "gene_name": "Uncharacterized protein FAM120AOS",
  "gene_symbol": "FAM120AOS",
  "term_id": "UNKNOWN:0002"
}